{
  "term_label": "Unknown biological process",
  "gene_symbol": "Q8N9W7",
  "gene": "UniProtKB:Q8N9W7",
  "gene_name": "Putative transmembrane protein FLJ36131",
  "term_id": "UNKNOWN:0002"
}